{
  "gene_symbol": "GPR108",
  "term_label": "Golgi apparatus",
  "term_id": "GO:0005794",
  "gene": "UniProtKB:Q9NPR9",
  "gene_name": "Protein GPR108"
}